{
  "gene": "UniProtKB:Q6P2Q9",
  "gene_name": "Pre-mRNA-processing-splicing factor 8",
  "gene_symbol": "PRPF8",
  "term_id": "GO:0017070",
  "term_label": "U6 snRNA binding"
}